{
  "gene": "UniProtKB:Q6PJT7",
  "gene_name": "Zinc finger CCCH domain-containing protein 14",
  "gene_symbol": "ZC3H14",
  "term_id": "GO:0005737",
  "term_label": "cytoplasm"
}